biogenic amine biosynthetic process [GO:0042401] (biological process) Definition: The chemical reactions and pathways occurring at the level of individual cells resulting in the formation of any of a group of naturally occurring, biologically active amines, such as norepinephrine, histamine, and serotonin, many of which act as neurotransmitters. Sources: GOC:jl, ISBN:0395825172 Relationships: is a type of biogenic amine metabolic process [GO:0006576]; is a type of amine biosynthetic process [GO:0009309] Subtypes: histamine biosynthetic process [GO:0001694], GO:0006589, polyamine biosynthetic process [GO:0006596], nicotianamine biosynthetic process [GO:0030418], GO:0042423, choline biosynthetic process [GO:0042425], GO:0042444, GO:0046219, ethanolamine biosynthetic process [GO:0046335] Also known as: biogenic amine anabolism, biogenic amine biosynthesis, biogenic amine formation, biogenic amine synthesis, cellular biogenic amine biosynthetic process